mitochondrial proton-transporting ATP synthase complex binding [GO:0140260] (MF) References: PMID:12110673 Relationships: is a type of protein-containing complex binding [GO:0044877] Definition: Binding to a mitochondrial proton-transporting ATP synthase complex.